triglyceride biosynthetic process [GO:0019432] (biological process) Regulation: regulated by regulation of triglyceride biosynthetic process [GO:0010866]; positively regulated by positive regulation of triglyceride biosynthetic process [GO:0010867]; negatively regulated by negative regulation of triglyceride biosynthetic process [GO:0010868] Sources: ISBN:0198506732 Also known as: triacylglycerol biosynthesis, triacylglycerol biosynthetic process, triglyceride anabolism, triglyceride biosynthesis, triglyceride formation, triglyceride synthesis Definition: The chemical reactions and pathways resulting in the formation of a triglyceride, any triester of glycerol. Relationships: is a type of triglyceride metabolic process [GO:0006641]; is a type of GO:0046463